{
  "gene": "UniProtKB:P62820",
  "gene_symbol": "RAB1A",
  "term_label": "endomembrane system",
  "gene_name": "Ras-related protein Rab-1A",
  "term_id": "GO:0012505"
}